{
  "term_id": "GO:0000978",
  "gene": "UniProtKB:Q8WUU4",
  "gene_name": "Zinc finger protein 296",
  "term_label": "RNA polymerase II cis-regulatory region sequence-specific DNA binding",
  "gene_symbol": "ZNF296"
}